{
  "gene_symbol": "FKBP10",
  "gene_name": "Peptidyl-prolyl cis-trans isomerase FKBP10",
  "gene": "UniProtKB:Q96AY3",
  "term_label": "endoplasmic reticulum",
  "term_id": "GO:0005783"
}